{
  "term_id": "UNKNOWN:0002",
  "gene": "UniProtKB:A0A1B0GTK5",
  "gene_symbol": "FAM236D",
  "term_label": "Unknown biological process",
  "gene_name": "Protein FAM236D"
}